response to cell size control checkpoint signaling [GO:0072470] (biological process) Also known as: cell size control checkpoint effector process, response to mitotic cell cycle cell size control checkpoint signaling, response to signal involved in cell size control checkpoint Definition: A process that occurs in response to signals generated as a result of cell size control checkpoint signaling. Sources: GOC:mtg_cell_cycle Subtypes: response to G1 cell size control checkpoint signaling [GO:0072449], response to G2 transition size control checkpoint signaling [GO:0072452] Relationships: is a type of response to mitotic cell cycle checkpoint signaling [GO:0072414]